{
  "term_label": "regulation of transcription by RNA polymerase II",
  "gene_name": "Zinc finger protein 250",
  "term_id": "GO:0006357",
  "gene_symbol": "ZNF250",
  "gene": "UniProtKB:P15622"
}